{
  "gene_symbol": "LRIT1",
  "gene_name": "Leucine-rich repeat, immunoglobulin-like domain and transmembrane domain-containing protein 1",
  "term_label": "Unknown molecular function",
  "gene": "UniProtKB:Q9P2V4",
  "term_id": "UNKNOWN:0001"
}